glutaconyl-CoA decarboxylase activity [GO:0018801] (molecular function) Definition: Catalysis of the reaction: trans-glutaconyl-CoA + H+ = but-2-enoyl-CoA + CO2. Relationships: is a type of decarboxylation-driven active transmembrane transporter activity [GO:0015451]; is a type of carboxy-lyase activity [GO:0016831] References: PMID:11248185 Sources: RHEA:23972 Also known as: 4-carboxybut-2-enoyl-CoA carboxy-lyase (but-2-enoyl-CoA-forming), 4-carboxybut-2-enoyl-CoA carboxy-lyase activity, glutaconyl coenzyme A decarboxylase activity, pent-2-enoyl-CoA carboxy-lyase activity